{
  "term_label": "nucleus",
  "term_id": "GO:0005634",
  "gene_symbol": "HOXD3",
  "gene_name": "Homeobox protein Hox-D3",
  "gene": "UniProtKB:P31249"
}